caffeate 3,4-dioxygenase activity [GO:0047762] (molecular function) Sources: EC:1.13.11.22, RHEA:22216 Definition: Catalysis of the reaction: trans-caffeate + O2 = 3-(2-carboxyethenyl)-cis,cis-muconate + 2 H+. Also known as: 3,4-dihydroxy-trans-cinnamate:oxygen 3,4-oxidoreductase (decyclizing) Relationships: is a type of oxidoreductase activity, acting on single donors with incorporation of molecular oxygen, incorporation of two atoms of oxygen [GO:0016702]